{
  "gene_symbol": "PGAP3",
  "term_id": "GO:0006506",
  "term_label": "GPI anchor biosynthetic process",
  "gene_name": "Post-GPI attachment to proteins factor 3",
  "gene": "UniProtKB:Q96FM1"
}